{
  "gene": "UniProtKB:Q8N0V5",
  "gene_symbol": "GCNT2",
  "term_id": "GO:0007179",
  "term_label": "transforming growth factor beta receptor signaling pathway",
  "gene_name": "N-acetyllactosaminide beta-1,6-N-acetylglucosaminyl-transferase"
}